{
  "term_id": "GO:0004520",
  "gene_symbol": "ERCC5",
  "gene": "UniProtKB:P28715",
  "term_label": "DNA endonuclease activity",
  "gene_name": "DNA excision repair protein ERCC-5"
}